pyridoxal oxidase activity [GO:0004732] (molecular function) Definition: Catalysis of the reaction:  pyridoxal + H2O + O2 = 4-pyridoxate + H+ + H2O2. Sources: RHEA:23724 Also known as: pyridoxal:oxygen 4-oxidoreductase activity Relationships: is a type of aldehyde oxidase activity [GO:0004031]